metanephric DCT cell development [GO:0072241] (biological process) Also known as: metanephric distal convoluted tubule cell development Definition: The process whose specific outcome is the progression of a metanephric distal convoluted tubule cell over time, from its formation to the mature structure. Sources: GOC:mtg_kidney_jan10 Relationships: is a type of DCT cell development [GO:0072140]; is part of GO:0072240